otic placode development [GO:1905040] (biological process) References: PMID:18356247 Sources: GOC:PARL, GOC:TermGenie, GOC:bf, GOC:mat, GO_REF:0000094 Also known as: placoda otica development, auditory placode development, ear placode development, ear/otic placode development, octaval VIII placode development, octaval placode development Relationships: is a type of ectodermal placode development [GO:0071696] Definition: The process whose specific outcome is the progression of an otic placode over time, from its formation to the mature structure.